{
  "gene_symbol": "DBX2",
  "gene_name": "Homeobox protein DBX2",
  "term_label": "regulation of transcription by RNA polymerase II",
  "gene": "UniProtKB:Q6ZNG2",
  "term_id": "GO:0006357"
}